{
  "gene_name": "Inositol hexakisphosphate kinase 2",
  "term_id": "GO:0005634",
  "term_label": "nucleus",
  "gene_symbol": "IP6K2",
  "gene": "UniProtKB:Q9UHH9"
}